{
  "gene": "UniProtKB:P53365",
  "term_id": "GO:0032588",
  "gene_name": "Arfaptin-2",
  "term_label": "trans-Golgi network membrane",
  "gene_symbol": "ARFIP2"
}